{
  "gene_symbol": "HSD3B1",
  "gene_name": "3 beta-hydroxysteroid dehydrogenase_Delta 5--4-isomerase type 1",
  "gene": "UniProtKB:P14060",
  "term_label": "steroid biosynthetic process",
  "term_id": "GO:0006694"
}